{
  "term_id": "UNKNOWN:0001",
  "gene_symbol": "TMEM273",
  "term_label": "Unknown molecular function",
  "gene": "UniProtKB:Q5T292",
  "gene_name": "Transmembrane protein 273"
}